{
  "term_label": "Unknown biological process",
  "gene": "UniProtKB:Q15057",
  "gene_symbol": "ACAP2",
  "term_id": "UNKNOWN:0002",
  "gene_name": "Arf-GAP with coiled-coil, ANK repeat and PH domain-containing protein 2"
}